cell cycle switching, mitotic to meiotic cell cycle [GO:0051728] (biological process) Sources: GOC:ai, GOC:mtg_cell_cycle Subtypes: GO:0051729 Definition: The process in which a cell switches cell cycle mode from mitotic to meiotic division. Also known as: conversion to meiotic cell cycle, entry into meiotic cell cycle, initiation of meiotic cell cycle, cell cycle switching, mitosis to meiosis, conversion to meiosis, entry into meiosis, initiation of meiosis, meiotic entry Regulation: regulated by regulation of cell cycle switching, mitotic to meiotic cell cycle [GO:0110044]; negatively regulated by negative regulation of cell cycle switching, mitotic to meiotic cell cycle [GO:0110045]; positively regulated by GO:0140648 Relationships: is a type of GO:0045930; is a type of positive regulation of meiotic cell cycle [GO:0051446]; is a type of GO:0060184